{
  "gene": "UniProtKB:Q9BYU1",
  "term_id": "GO:0048666",
  "gene_symbol": "PBX4",
  "term_label": "neuron development",
  "gene_name": "Pre-B-cell leukemia transcription factor 4"
}